{
  "gene_symbol": "TARDBP",
  "term_label": "nucleoplasm",
  "gene": "UniProtKB:Q13148",
  "term_id": "GO:0005654",
  "gene_name": "TAR DNA-binding protein 43"
}